{
  "gene": "UniProtKB:Q7L8A9",
  "term_id": "GO:0005737",
  "gene_name": "Tubulinyl-Tyr carboxypeptidase 1",
  "term_label": "cytoplasm",
  "gene_symbol": "VASH1"
}